{
  "gene_symbol": "ZNF749",
  "gene_name": "Zinc finger protein 749",
  "term_label": "regulation of transcription by RNA polymerase II",
  "term_id": "GO:0006357",
  "gene": "UniProtKB:O43361"
}